{
  "gene": "UniProtKB:P12524",
  "term_label": "RNA polymerase II cis-regulatory region sequence-specific DNA binding",
  "gene_symbol": "MYCL",
  "gene_name": "Protein L-Myc",
  "term_id": "GO:0000978"
}